{
  "gene_name": "Protein mono-ADP-ribosyltransferase PARP3",
  "term_label": "double-strand break repair",
  "gene": "UniProtKB:Q9Y6F1",
  "term_id": "GO:0006302",
  "gene_symbol": "PARP3"
}